{
  "gene_name": "MTRF1L release factor glutamine methyltransferase",
  "gene": "UniProtKB:Q9Y5R4",
  "term_id": "GO:0036009",
  "gene_symbol": "HEMK1",
  "term_label": "protein-glutamine N-methyltransferase activity"
}